polyamine transport [GO:0015846] (biological process) Relationships: is a type of nitrogen compound transport [GO:0071705] Sources: GOC:krc, ISBN:0198506732 Subtypes: spermine transport [GO:0000296], putrescine transport [GO:0015847], GO:0015848, polyamine transmembrane transport [GO:1902047] Definition: The directed movement of polyamines, organic compounds containing two or more amino groups, into, out of or within a cell, or between cells, by means of some agent such as a transporter or pore.